IAA-Phe conjugate hydrolase activity [GO:0010210] (molecular function) Sources: GOC:syr Relationships: is a type of GO:0010178 Definition: Catalysis of the reaction: indole-3-acetyl-phenylalanine + H2O = indole-3-acetate + phenylalanine.